histone H2AK13 ubiquitin ligase activity [GO:0140856] (molecular function) Note: Note that the residue position corresponds to the canonical human H2A2A histone (UniProtKB:Q6FI13); this residue is conserved across all eukaryotes. Residue 1 is the first residue following removal of the initiating Methionine (Met). Note that each histone is encoded by multiple genes, and sequences may vary across different genes within an organism. Relationships: is a type of GO:0141053 References: PMID:22980979, PMID:28624371 Definition: Catalysis of the transfer of a ubiquitin molecule to histone 2A at the lysine-13 residue. Also known as: histone ubiquitin ligase activity (H2A-K13 specific)